positive regulation of brood size [GO:0090727] (biological process) Sources: GOC:rz Relationships: is a type of GO:0065007 Definition: Any process that increases brood size. Brood size is the number of progeny that survive embryogenesis and are cared for at one time.